{
  "gene": "UniProtKB:Q9BX46",
  "term_label": "cytosol",
  "gene_symbol": "RBM24",
  "term_id": "GO:0005829",
  "gene_name": "RNA-binding protein 24"
}